{
  "gene_name": "Protein-glutamine gamma-glutamyltransferase 4",
  "term_label": "extracellular matrix",
  "gene": "UniProtKB:P49221",
  "term_id": "GO:0031012",
  "gene_symbol": "TGM4"
}